{
  "gene_name": "Steroid receptor-associated and regulated protein",
  "gene_symbol": "SRARP",
  "gene": "UniProtKB:Q8NEQ6",
  "term_label": "positive regulation of intracellular estrogen receptor signaling pathway",
  "term_id": "GO:0033148"
}